{
  "gene": "UniProtKB:Q15111",
  "gene_symbol": "PLCL1",
  "term_label": "regulation of synaptic transmission, GABAergic",
  "gene_name": "Inactive phospholipase C-like protein 1",
  "term_id": "GO:0032228"
}